{
  "gene": "UniProtKB:P16389",
  "gene_name": "Potassium voltage-gated channel subfamily A member 2",
  "term_id": "GO:0030425",
  "gene_symbol": "KCNA2",
  "term_label": "dendrite"
}